{
  "term_id": "GO:0030672",
  "gene": "UniProtKB:Q9HC10",
  "term_label": "synaptic vesicle membrane",
  "gene_symbol": "OTOF",
  "gene_name": "Otoferlin"
}